polyadenylation-dependent RNA catabolic process [GO:0043633] (BP) Definition: The chemical reactions and pathways resulting in the breakdown of an RNA molecule, initiated by the enzymatic addition of a sequence of adenylyl residues (polyadenylation) at the 3'-end of the target RNA. Sources: GOC:dgf, GOC:jl, GOC:krc Relationships: is a type of RNA catabolic process [GO:0006401]; is a type of GO:0043632 Subtypes: GO:0043634, cytoplasmic polyadenylation-dependent RNA catabolic process [GO:0180018]